{
  "term_id": "GO:0005737",
  "gene_name": "E3 ubiquitin-protein ligase TRIM32",
  "gene_symbol": "TRIM32",
  "gene": "UniProtKB:Q13049",
  "term_label": "cytoplasm"
}